malate dehydrogenase activity [GO:0016615] (molecular function) Sources: GOC:mah, ISBN:0582227089 Subtypes: malic enzyme activity [GO:0004470], L-malate dehydrogenase (quinone) activity [GO:0008924], GO:0030060, GO:0046553, L-malate dehydrogenase (NADP+) activity [GO:0046554] Definition: Catalysis of the reversible conversion of pyruvate or oxaloacetate to malate. Relationships: is a type of oxidoreductase activity, acting on CH-OH group of donors [GO:0016614]